{
  "gene_name": "Catenin beta-1",
  "gene_symbol": "CTNNB1",
  "term_label": "adherens junction",
  "term_id": "GO:0005912",
  "gene": "UniProtKB:P35222"
}